{
  "term_id": "GO:0045944",
  "gene_name": "Akirin-2",
  "term_label": "positive regulation of transcription by RNA polymerase II",
  "gene_symbol": "AKIRIN2",
  "gene": "UniProtKB:Q53H80"
}